UV-A, blue light phototransduction [GO:0009588] (biological process) Also known as: blue-sensitive opsin, short-wave-sensitive opsin, violet-sensitive opsin Definition: The sequence of reactions within a cell required to convert absorbed photons from UV-A or blue light into a molecular signal; the UV-A, blue light range is defined as having a wavelength within the range of 315 to 400 nm. Relationships: is a type of phototransduction [GO:0007602] Sources: GOC:mah